{
  "gene_name": "Putative uncharacterized protein encoded by LINC00523",
  "gene_symbol": "LINC00523",
  "term_label": "Unknown cellular component",
  "gene": "UniProtKB:Q86TU6",
  "term_id": "UNKNOWN:0003"
}